{
  "gene_symbol": "NOTCH3",
  "gene": "UniProtKB:Q9UM47",
  "term_id": "UNKNOWN:0001",
  "term_label": "Unknown molecular function",
  "gene_name": "Neurogenic locus notch homolog protein 3"
}